{
  "term_label": "glutamate metabolic process",
  "term_id": "GO:0006536",
  "gene_symbol": "NAGS",
  "gene": "UniProtKB:Q8N159",
  "gene_name": "N-acetylglutamate synthase, mitochondrial"
}